{
  "term_id": "UNKNOWN:0001",
  "gene": "UniProtKB:Q8IYG6",
  "term_label": "Unknown molecular function",
  "gene_symbol": "LRRC56",
  "gene_name": "Leucine-rich repeat-containing protein 56"
}